{
  "term_label": "protein ubiquitination",
  "gene_symbol": "UHRF1",
  "gene_name": "E3 ubiquitin-protein ligase UHRF1",
  "gene": "UniProtKB:Q96T88",
  "term_id": "GO:0016567"
}